{
  "term_label": "AMP deaminase activity",
  "term_id": "GO:0003876",
  "gene_symbol": "AMPD2",
  "gene_name": "AMP deaminase 2",
  "gene": "UniProtKB:Q01433"
}